{
  "gene_symbol": "MRFAP1L1",
  "gene": "UniProtKB:Q96HT8",
  "term_label": "Unknown cellular component",
  "term_id": "UNKNOWN:0003",
  "gene_name": "MORF4 family-associated protein 1-like 1"
}